{
  "gene_name": "Lysophosphatidylcholine acyltransferase 2",
  "gene": "UniProtKB:Q7L5N7",
  "gene_symbol": "LPCAT2",
  "term_label": "lysophosphatidic acid acyltransferase activity",
  "term_id": "GO:0042171"
}